coniferyl-alcohol glucosyltransferase activity [GO:0047209] (molecular function) Relationships: is a type of UDP-glucosyltransferase activity [GO:0035251] Also known as: UDP-glucose coniferyl alcohol glucosyltransferase activity, UDP-glucose:coniferyl-alcohol 4'-beta-D-glucosyltransferase activity, UDPglucose:coniferyl-alcohol 4'-beta-D-glucosyltransferase activity, uridine diphosphoglucose-coniferyl alcohol glucosyltransferase activity Sources: EC:2.4.1.111, MetaCyc:2.4.1.111-RXN Definition: Catalysis of the reaction: coniferyl alcohol + UDP-D-glucose = coniferin + UDP.